{
  "gene_name": "LHFPL tetraspan subfamily member 3 protein",
  "term_id": "GO:0007605",
  "term_label": "sensory perception of sound",
  "gene_symbol": "LHFPL3",
  "gene": "UniProtKB:Q86UP9"
}